symbiont-mediated suppression of host exocytosis [GO:0141157] (biological process) Definition: A process in which a symbiont inhibits or disrupts the normal execution of  host exocytosis. The host is defined as the larger of the organisms involved in a symbiotic interaction. References: PMID:17185412 Relationships: is a type of symbiont-mediated perturbation of host vesicle-mediated transport [GO:1990215]